{
  "gene": "UniProtKB:O60503",
  "term_label": "cAMP biosynthetic process",
  "term_id": "GO:0006171",
  "gene_symbol": "ADCY9",
  "gene_name": "Adenylate cyclase type 9"
}